rRNA processing [GO:0006364] (biological process) Relationships: is a type of RNA processing [GO:0006396]; is a type of rRNA metabolic process [GO:0016072]; is part of ribosome biogenesis [GO:0042254] Definition: Any process involved in the conversion of a primary ribosomal RNA (rRNA) transcript into one or more mature rRNA molecules. Subtypes: rRNA modification [GO:0000154], endonucleolytic cleavage of tricistronic rRNA transcript (SSU-rRNA, LSU-rRNA, 5S) [GO:0000449], cleavage of bicistronic rRNA transcript (SSU-rRNA, LSU-rRNA) [GO:0000450], GO:0000460, GO:0000470, maturation of 2S rRNA [GO:0000475], maturation of 4.5S rRNA [GO:0000476], endonucleolytic cleavage of tricistronic rRNA transcript (SSU-rRNA, 5.8S rRNA, LSU-rRNA) [GO:0000479], GO:0000481, endonucleolytic cleavage of tetracistronic rRNA transcript (SSU-rRNA, 5.8S rRNA, 2S rRNA, LSU-rRNA) [GO:0000483], rRNA 5'-end processing [GO:0000967], endonucleolytic cleavage of tetracistronic rRNA transcript (SSU-rRNA, LSU-rRNA, 4.5S-rRNA, 5S-rRNA) [GO:0002103], maturation of SSU-rRNA [GO:0030490], rRNA 3'-end processing [GO:0031125], GO:1901259, snoRNA release from pre-rRNA [GO:1990417] Regulation: regulated by GO:2000232; negatively regulated by negative regulation of rRNA processing [GO:2000233]; positively regulated by positive regulation of rRNA processing [GO:2000234] Also known as: 35S primary transcript processing Sources: GOC:curators